L-cysteine catabolic process to hypotaurine [GO:0019449] (biological process) Definition: The chemical reactions and pathways resulting in the breakdown of L-cysteine into other compounds, including hypotaurine. Sources: GOC:go_curators Also known as: L-cysteine breakdown to hypotaurine, L-cysteine degradation to hypotaurine Relationships: is a type of L-cysteine catabolic process [GO:0019448]